{
  "gene_symbol": "ARFGEF2",
  "term_id": "GO:0005085",
  "gene_name": "Brefeldin A-inhibited guanine nucleotide-exchange protein 2",
  "gene": "UniProtKB:Q9Y6D5",
  "term_label": "guanyl-nucleotide exchange factor activity"
}